{
  "gene": "UniProtKB:Q3T906",
  "gene_symbol": "GNPTAB",
  "term_label": "N-glycan processing to lysosome",
  "term_id": "GO:0016256",
  "gene_name": "N-acetylglucosamine-1-phosphotransferase subunits alpha_beta"
}